Delta24(24-1) sterol reductase activity [GO:0000246] (molecular function) Relationships: is a type of oxidoreductase activity, acting on the CH-CH group of donors, NAD or NADP as acceptor [GO:0016628] Also known as: D24(24-1)-sterol reductase activity, sterol delta-24(28) methylene reductase activity, sterol delta-24(28) reductase activity, C-24(28) sterol reductase activity, delta24(241)-sterol reductase activity, ergosterol:NADP+ delta24(241)-oxidoreductase activity, sterol Delta(24(28))-methylene reductase activity, sterol Delta(24(28))-reductase activity, sterol delta24(28)-methylene reductase activity, sterol delta24(28)-reductase activity Sources: EC:1.3.1.71, RHEA:18501 Definition: Catalysis of the reaction: ergosterol + NADP+ = ergosta-5,7,22,24(24(1))-tetraen-3beta-ol + H+ + NADPH.